{
  "gene_symbol": "PNMA6F",
  "term_id": "UNKNOWN:0002",
  "gene": "UniProtKB:A0A0J9YX94",
  "term_label": "Unknown biological process",
  "gene_name": "Paraneoplastic antigen Ma6F"
}